{
  "term_id": "UNKNOWN:0002",
  "term_label": "Unknown biological process",
  "gene": "UniProtKB:Q8NH42",
  "gene_symbol": "OR4K13",
  "gene_name": "Olfactory receptor 4K13"
}